{
  "term_label": "oxidoreductase activity, acting on the CH-OH group of donors, NAD or NADP as acceptor",
  "gene_name": "Sterol-4-alpha-carboxylate 3-dehydrogenase, decarboxylating",
  "gene": "UniProtKB:Q15738",
  "term_id": "GO:0016616",
  "gene_symbol": "NSDHL"
}